{
  "term_label": "neuron differentiation",
  "gene_symbol": "LHX3",
  "term_id": "GO:0030182",
  "gene": "UniProtKB:Q9UBR4",
  "gene_name": "LIM_homeobox protein Lhx3"
}